{
  "gene": "UniProtKB:Q4G0S7",
  "term_id": "UNKNOWN:0002",
  "gene_name": "Coiled-coil domain-containing protein 152",
  "gene_symbol": "CCDC152",
  "term_label": "Unknown biological process"
}